{
  "gene": "UniProtKB:Q9H1C0",
  "term_id": "UNKNOWN:0001",
  "gene_name": "Lysophosphatidic acid receptor 5",
  "gene_symbol": "LPAR5",
  "term_label": "Unknown molecular function"
}